{
  "term_label": "RNA polymerase II cis-regulatory region sequence-specific DNA binding",
  "term_id": "GO:0000978",
  "gene_name": "Zinc finger protein 580",
  "gene": "UniProtKB:Q9UK33",
  "gene_symbol": "ZNF580"
}